{
  "gene_name": "Potassium channel subfamily T member 1",
  "gene_symbol": "KCNT1",
  "term_id": "GO:0071805",
  "gene": "UniProtKB:Q5JUK3",
  "term_label": "potassium ion transmembrane transport"
}